{
  "gene": "UniProtKB:Q86WC4",
  "term_label": "Unknown molecular function",
  "gene_name": "Osteopetrosis-associated transmembrane protein 1",
  "gene_symbol": "OSTM1",
  "term_id": "UNKNOWN:0001"
}